regulation of eosinophil degranulation [GO:0043309] (biological process) Sources: ISBN:0781735149 Subtypes: negative regulation of eosinophil degranulation [GO:0043310], GO:0043311 Also known as: regulation of eosinophil granule exocytosis Definition: Any process that modulates the frequency, rate, or extent of eosinophil degranulation. Relationships: is a type of regulation of myeloid leukocyte mediated immunity [GO:0002886]; is a type of regulation of leukocyte degranulation [GO:0043300]; is a type of regulation of immune response [GO:0050776]; regulates eosinophil degranulation [GO:0043308]